{
  "gene": "UniProtKB:Q5HYK7",
  "term_label": "cytoskeleton organization",
  "gene_name": "SH3 domain-containing protein 19",
  "term_id": "GO:0007010",
  "gene_symbol": "SH3D19"
}